arabinonate dehydratase activity [GO:0047675] (molecular function) Relationships: is a type of hydro-lyase activity [GO:0016836] Also known as: D-arabinonate hydro-lyase (2-dehydro-3-deoxy-D-arabinonate-forming), D-arabinonate hydro-lyase activity Sources: EC:4.2.1.5, RHEA:21836 Definition: Catalysis of the reaction: D-arabinonate = 2-dehydro-3-deoxy-D-arabinonate + H2O.